{
  "gene_name": "Putative WASP homolog-associated protein with actin, membranes and microtubules-like protein 1",
  "gene_symbol": "WHAMMP3",
  "term_label": "Unknown molecular function",
  "term_id": "UNKNOWN:0001",
  "gene": "UniProtKB:Q1A5X7"
}